{
  "gene_symbol": "CMPK2",
  "term_label": "dTTP biosynthetic process",
  "gene": "UniProtKB:Q5EBM0",
  "term_id": "GO:0006235",
  "gene_name": "UMP-CMP kinase 2, mitochondrial"
}